{
  "term_id": "GO:0008021",
  "gene": "UniProtKB:P23560",
  "gene_name": "Brain-derived neurotrophic factor",
  "term_label": "synaptic vesicle",
  "gene_symbol": "BDNF"
}